bile-acid-CoA transferase activity [GO:0033881] (MF) Definition: Catalysis of the reaction: deoxycholoyl-CoA + cholate = deoxycholate + choloyl-CoA. Also known as: bile-acid-CoA hydrolase activity, deoxycholoyl-CoA transferase activity Relationships: is a type of GO:0008410 References: PMID:22021638 Sources: RHEA:49436